{
  "term_id": "UNKNOWN:0001",
  "gene": "UniProtKB:A0A0K0K1G8",
  "gene_symbol": "TRBV10-2",
  "gene_name": "T cell receptor beta variable 10-2",
  "term_label": "Unknown molecular function"
}